C-acetyltransferase activity [GO:0016453] (molecular function) Definition: Catalysis of the transfer of an acetyl group to a carbon atom on the acceptor molecule. Relationships: is a type of acetyltransferase activity [GO:0016407]; is a type of C-acyltransferase activity [GO:0016408] Sources: GOC:ai Subtypes: acetyl-CoA C-acetyltransferase activity [GO:0003985], GO:0008861, glycine C-acetyltransferase activity [GO:0008890]